oxidoreductase activity, acting on the CH-NH group of donors, flavin as acceptor [GO:0046997] (molecular function) Subtypes: GO:0008480, dimethylamine dehydrogenase activity [GO:0047133], GO:0047865, trimethylamine dehydrogenase activity [GO:0050470] Sources: GOC:jl Definition: Catalysis of an oxidation-reduction (redox) reaction in which a CH-NH group acts as a hydrogen or electron donor and reduces a flavin. Relationships: is a type of oxidoreductase activity, acting on the CH-NH group of donors [GO:0016645]